{
  "term_label": "Unknown molecular function",
  "term_id": "UNKNOWN:0001",
  "gene_symbol": "PNMA5",
  "gene_name": "Paraneoplastic antigen-like protein 5",
  "gene": "UniProtKB:Q96PV4"
}